{
  "gene_symbol": "AGTRAP",
  "gene_name": "Type-1 angiotensin II receptor-associated protein",
  "gene": "UniProtKB:Q6RW13",
  "term_label": "Unknown molecular function",
  "term_id": "UNKNOWN:0001"
}